histone H1N76/N77 asparagine deamidase activity [GO:0160264] (MF) Definition: Catalysis of the reaction: histone H1 L-asparagine [positions 76 and 77] + H2O = histone H1 L-aspartate [positions 76 and 77] + NH4+. References: PMID:40240600 Relationships: is a type of histone H1 asparagine deamidase activity [GO:0160261]